platelet-derived growth factor production [GO:0090360] (biological process) Relationships: is a type of cytokine production [GO:0001816] Definition: The appearance of any platelet-derived growth factor due to biosynthesis or secretion following a cellular stimulus, resulting in an increase in its intracellular or extracellular levels. Note: Note that this term is in the subset of terms that should not be used for direct gene product annotation. Instead, select one of the 'regulation' children terms. Sources: GOC:BHF Regulation: regulated by regulation of platelet-derived growth factor production [GO:0090361]; positively regulated by GO:0090362